{
  "gene_symbol": "PTTG1IP2",
  "term_id": "UNKNOWN:0002",
  "gene_name": "PTTG1IP family member 2",
  "term_label": "Unknown biological process",
  "gene": "UniProtKB:P0DTF9"
}